{
  "gene_name": "Cyclin-dependent kinase 2-associated protein 2",
  "term_id": "GO:0005874",
  "term_label": "microtubule",
  "gene": "UniProtKB:O75956",
  "gene_symbol": "CDK2AP2"
}